{
  "gene_name": "Complement factor H-related protein 3",
  "gene_symbol": "CFHR3",
  "term_id": "GO:0001851",
  "term_label": "complement component C3b binding",
  "gene": "UniProtKB:Q02985"
}